{
  "gene_name": "Cilia- and flagella-associated protein 61",
  "gene_symbol": "CFAP61",
  "gene": "UniProtKB:Q8NHU2",
  "term_label": "sperm flagellum",
  "term_id": "GO:0036126"
}